nematode pharyngeal gland morphogenesis [GO:1905905] (biological process) References: PMID:21868609 Sources: GOC:TermGenie, GO_REF:0000083 Also known as: pharynx gland morphogenesis, glandulae pharyngeae morphogenesis Definition: The developmental process by which a nematode pharyngeal gland is generated and organized. Relationships: is a type of anatomical structure morphogenesis [GO:0009653]